{
  "term_id": "GO:0005886",
  "gene_symbol": "CD37",
  "gene_name": "Leukocyte antigen CD37",
  "term_label": "plasma membrane",
  "gene": "UniProtKB:P11049"
}